lysine biosynthetic process via diaminopimelate, dehydrogenase pathway [GO:0033361] (biological process) Relationships: is a type of lysine biosynthetic process via diaminopimelate [GO:0009089]; BFO_0000051 diaminopimelate dehydrogenase activity [GO:0047850] Sources: GOC:mah, GOC:pr, MetaCyc:PWY-2942 Definition: The chemical reactions and pathways resulting in the formation of lysine, via the intermediate diaminopimelate; in this pathway tetrahydrodipicolinate is converted to meso-diaminopimelate in a single enzymatic step. Also known as: lysine anabolism via diaminopimelate, dehydrogenase pathway, lysine biosynthesis via diaminopimelic acid, dehydrogenase pathway, lysine formation via diaminopimelate, dehydrogenase pathway, lysine synthesis via diaminopimelate, dehydrogenase pathway